{
  "term_label": "cytoplasm",
  "gene_symbol": "NOVA1",
  "gene_name": "RNA-binding protein Nova-1",
  "term_id": "GO:0005737",
  "gene": "UniProtKB:P51513"
}